{
  "term_id": "UNKNOWN:0001",
  "gene_symbol": "Q6ZS46",
  "term_label": "Unknown molecular function",
  "gene": "UniProtKB:Q6ZS46",
  "gene_name": "Putative uncharacterized protein FLJ45840"
}